{
  "term_label": "protein ubiquitination",
  "gene": "UniProtKB:Q96PU4",
  "term_id": "GO:0016567",
  "gene_name": "E3 ubiquitin-protein ligase UHRF2",
  "gene_symbol": "UHRF2"
}